{
  "gene_name": "Putative dispanin subfamily A member 2d",
  "term_label": "response to interferon-alpha",
  "term_id": "GO:0035455",
  "gene_symbol": "C9JQL5",
  "gene": "UniProtKB:C9JQL5"
}